{
  "gene_name": "Polypeptide N-acetylgalactosaminyltransferase 9",
  "term_label": "protein O-linked glycosylation",
  "term_id": "GO:0006493",
  "gene": "UniProtKB:Q9HCQ5",
  "gene_symbol": "GALNT9"
}